{
  "gene_name": "Homeobox protein Hox-D8",
  "term_id": "GO:0000981",
  "gene_symbol": "HOXD8",
  "term_label": "DNA-binding transcription factor activity, RNA polymerase II-specific",
  "gene": "UniProtKB:P13378"
}